{
  "gene_name": "Killer cell immunoglobulin-like receptor 2DL1",
  "gene_symbol": "KIR2DL1",
  "term_label": "immune response-inhibiting cell surface receptor signaling pathway",
  "term_id": "GO:0002767",
  "gene": "UniProtKB:P43626"
}